{
  "gene_name": "Dual specificity tyrosine-phosphorylation-regulated kinase 1B",
  "gene_symbol": "DYRK1B",
  "gene": "UniProtKB:Q9Y463",
  "term_label": "nucleus",
  "term_id": "GO:0005634"
}